{
  "gene": "UniProtKB:Q9Y247",
  "term_label": "chromatin organization",
  "gene_symbol": "FAM50B",
  "gene_name": "Protein FAM50B",
  "term_id": "GO:0006325"
}